endochondral ossification [GO:0001958] (biological process) Relationships: is_a replacement ossification [GO:0036075]; is part of GO:0060350 Definition: Replacement ossification wherein bone tissue replaces cartilage. Sources: GO_REF:0000034, ISBN:0878932437